regulation of SNARE complex disassembly [GO:0035495] (BP) Relationships: is a type of regulation of protein-containing complex disassembly [GO:0043244]; regulates SNARE complex disassembly [GO:0035494] Subtypes: positive regulation of SNARE complex disassembly [GO:0035540], negative regulation of SNARE complex disassembly [GO:0035541] Definition: Any process that modulates the frequency, rate or extent of disassembly of the SNARE complex. The SNARE complex is a protein complex involved in membrane fusion; a stable ternary complex consisting of a four-helix bundle, usually formed from one R-SNARE and three Q-SNAREs with an ionic layer sandwiched between hydrophobic layers. Sources: GOC:rb